rhombomere 1 development [GO:0021567] (biological process) Definition: The process whose specific outcome is the progression of rhombomere 1 over time, from its formation to the mature structure. Rhombomeres are transverse segments of the developing rhombencephalon. Rhombomeres are lineage restricted, express different genes from one another, and adopt different developmental fates. Rhombomeres are numbered in anterior to posterior order. Sources: GOC:cls, GOC:curators, GOC:dgh, GOC:dph, GOC:jid Relationships: is a type of rhombomere development [GO:0021546]